{
  "term_label": "extracellular space",
  "gene_symbol": "PSPN",
  "gene": "UniProtKB:O60542",
  "term_id": "GO:0005615",
  "gene_name": "Persephin"
}